{
  "term_id": "GO:0005886",
  "term_label": "plasma membrane",
  "gene": "UniProtKB:Q14449",
  "gene_symbol": "GRB14",
  "gene_name": "Growth factor receptor-bound protein 14"
}